4-sulfomuconolactone hydrolase activity [GO:0102998] (molecular function) Sources: EC:3.1.1.92 Definition: Catalysis of the reaction: (5-oxo-2-sulfonato-2,5-dihydrofuran-2-yl)acetate + H2O = maleylacetate + sulfite + 2 H+. Relationships: is a type of carboxylic ester hydrolase activity [GO:0052689]